{
  "gene": "UniProtKB:Q16186",
  "term_id": "UNKNOWN:0002",
  "term_label": "Unknown biological process",
  "gene_symbol": "ADRM1",
  "gene_name": "Proteasomal ubiquitin receptor ADRM1"
}